heme O biosynthetic process [GO:0048034] (biological process) Also known as: haem O biosynthesis, haem O biosynthetic process, heme O anabolism, heme O biosynthesis, heme O formation, heme O synthesis Relationships: is a type of heme biosynthetic process [GO:0006783] Definition: The chemical reactions and pathways resulting in the formation of heme O, a derivative of heme containing a 17-carbon hydroxyethylfarnesyl side chain at position 8 of the tetrapyrrole macrocycle. Sources: GOC:jid